regulation of endosome size [GO:0051036] (biological process) Sources: GOC:ai Also known as: endosome enlargement Relationships: is a type of regulation of vesicle size [GO:0097494] Definition: Any process that modulates the volume of an endosome, a membrane-bounded organelle that carries materials newly ingested by endocytosis.